{
  "term_label": "plasma membrane",
  "gene_symbol": "SLC7A2",
  "term_id": "GO:0005886",
  "gene_name": "Cationic amino acid transporter 2",
  "gene": "UniProtKB:P52569"
}